{
  "term_id": "GO:0006974",
  "gene_name": "Serine_threonine-protein kinase WNK1",
  "term_label": "DNA damage response",
  "gene_symbol": "WNK1",
  "gene": "UniProtKB:Q9H4A3"
}